{
  "gene": "UniProtKB:Q9NPD8",
  "term_label": "DNA damage response",
  "gene_name": "Ubiquitin-conjugating enzyme E2 T",
  "term_id": "GO:0006974",
  "gene_symbol": "UBE2T"
}